MIS12/MIND type complex [GO:0000444] (cellular component) Relationships: is a type of outer kinetochore [GO:0000940] References: PMID:14633972, PMID:16585270 Sources: GOC:krc Definition: A multiprotein kinetochore subcomplex that binds to centromeric chromatin and forms part of the outer kinetochore. It helps to recruit outer kinetochore subunits that will bind to microtubules. In humans, it consists of MIS12, DSN1, NSL1 and PMF1. Also known as: MIND complex, Mis12 complex, Mtw1p Including Nnf1p-Nsl1p-Dsn1p complex, nuclear MIS12/MIND complex